{
  "gene_symbol": "ZSCAN30",
  "term_label": "regulation of transcription by RNA polymerase II",
  "gene": "UniProtKB:Q86W11",
  "gene_name": "Zinc finger and SCAN domain-containing protein 30",
  "term_id": "GO:0006357"
}